{
  "term_label": "cytoplasm",
  "term_id": "GO:0005737",
  "gene_name": "Pituitary tumor-transforming gene 1 protein-interacting protein",
  "gene_symbol": "PTTG1IP",
  "gene": "UniProtKB:P53801"
}